{
  "gene_symbol": "OR2W3",
  "term_label": "olfactory receptor activity",
  "gene_name": "Olfactory receptor 2W3",
  "gene": "UniProtKB:Q7Z3T1",
  "term_id": "GO:0004984"
}